{
  "gene_name": "Heat shock transcription factor, Y-linked",
  "gene": "UniProtKB:Q96LI6",
  "term_id": "GO:0005634",
  "gene_symbol": "HSFY2",
  "term_label": "nucleus"
}